{
  "term_id": "GO:0043063",
  "gene_symbol": "TEX14",
  "gene": "UniProtKB:Q8IWB6",
  "gene_name": "Inactive serine_threonine-protein kinase TEX14",
  "term_label": "intercellular bridge organization"
}